{
  "term_label": "membrane",
  "gene_symbol": "DGKQ",
  "gene": "UniProtKB:P52824",
  "gene_name": "Diacylglycerol kinase theta",
  "term_id": "GO:0016020"
}